{
  "gene_symbol": "MFN2",
  "term_id": "GO:0005741",
  "term_label": "mitochondrial outer membrane",
  "gene_name": "Mitofusin-2",
  "gene": "UniProtKB:O95140"
}